{
  "gene_name": "Calcium-independent phospholipase A2-gamma",
  "term_label": "calcium-independent phospholipase A2 activity",
  "term_id": "GO:0047499",
  "gene_symbol": "PNPLA8",
  "gene": "UniProtKB:Q9NP80"
}